{
  "gene_symbol": "TRBV5-5",
  "term_id": "UNKNOWN:0001",
  "gene_name": "T cell receptor beta variable 5-5",
  "term_label": "Unknown molecular function",
  "gene": "UniProtKB:A0A597"
}